{
  "term_label": "cytoplasm",
  "gene_name": "Stathmin domain-containing protein 1",
  "term_id": "GO:0005737",
  "gene": "UniProtKB:H3BQB6",
  "gene_symbol": "STMND1"
}